{
  "gene": "UniProtKB:Q6PDB4",
  "term_label": "nucleus",
  "term_id": "GO:0005634",
  "gene_name": "Zinc finger protein 880",
  "gene_symbol": "ZNF880"
}